{
  "gene_name": "Integrin beta-5",
  "term_label": "focal adhesion",
  "gene_symbol": "ITGB5",
  "term_id": "GO:0005925",
  "gene": "UniProtKB:P18084"
}